{
  "term_label": "regulation of centrosome cycle",
  "gene_symbol": "WDR62",
  "gene_name": "WD repeat-containing protein 62",
  "term_id": "GO:0046605",
  "gene": "UniProtKB:O43379"
}